female genitalia morphogenesis [GO:0048807] (biological process) Definition: The process in which the anatomical structures of female genitalia are generated and organized. Also known as: female genital morphogenesis Subtypes: GO:0048804 Relationships: is a type of genitalia morphogenesis [GO:0035112]; is part of female genitalia development [GO:0030540] Sources: GOC:mah